(R,S)-4-hydroxy-2-oxoglutarate aldolase activity [GO:0008700] (molecular function) Definition: Catalysis of the reaction: 4-hydroxy-2-oxoglutarate = pyruvate + glyoxylate. Can act on both the (4R) and the (4S) enantiomers of 4-hydroxy-2-oxoglutarate. Sources: EC:4.1.3.16, RHEA:18169 Also known as: 2-keto-4-hydroxyglutarate aldolase activity, 2-keto-4-hydroxybutyrate aldolase activity, 2-keto-4-hydroxyglutaric aldolase activity, 2-oxo-4-hydroxyglutarate aldolase activity, 2-oxo-4-hydroxyglutaric aldolase activity, 4-hydroxy-2-ketoglutarate aldolase activity, 4-hydroxy-2-ketoglutaric aldolase activity, 4-hydroxy-2-oxoglutarate glyoxylate-lyase (pyruvate-forming), 4-hydroxy-2-oxoglutarate glyoxylate-lyase activity, DL-4-hydroxy-2-ketoglutarate aldolase activity, KHG-aldolase activity, hydroxyketoglutarate aldolase activity, hydroxyketoglutaric aldolase activity Relationships: is a type of oxo-acid-lyase activity [GO:0016833]